{
  "term_id": "GO:0007178",
  "gene_name": "Inhibin beta C chain",
  "term_label": "cell surface receptor protein serine/threonine kinase signaling pathway",
  "gene": "UniProtKB:P55103",
  "gene_symbol": "INHBC"
}